{
  "gene_name": "Telomere repeats-binding bouquet formation protein 2",
  "term_label": "homologous chromosome pairing at meiosis",
  "gene_symbol": "TERB2",
  "term_id": "GO:0007129",
  "gene": "UniProtKB:Q8NHR7"
}